positive regulation of juvenile hormone biosynthetic process [GO:0045969] (biological process) Relationships: is a type of GO:0007557; is a type of positive regulation of hormone biosynthetic process [GO:0046886]; is a type of positive regulation of lipid biosynthetic process [GO:0046889]; positively regulates GO:0006718 Also known as: positive regulation of juvenile hormone anabolism, positive regulation of juvenile hormone biosynthesis, positive regulation of juvenile hormone formation, positive regulation of juvenile hormone synthesis, up regulation of juvenile hormone biosynthetic process, up-regulation of juvenile hormone biosynthetic process, upregulation of juvenile hormone biosynthetic process, activation of juvenile hormone biosynthetic process, stimulation of juvenile hormone biosynthetic process Sources: GOC:go_curators Definition: Any process that activates or increases the frequency, rate or extent of the chemical reactions and pathways resulting in the formation of juvenile hormone.